{
  "gene_name": "UDP-glucuronosyltransferase 1-6",
  "gene_symbol": "UGT1A6",
  "gene": "UniProtKB:P19224",
  "term_label": "flavone metabolic process",
  "term_id": "GO:0051552"
}